superoxide anion generation [GO:0042554] (biological process) Relationships: is a type of superoxide metabolic process [GO:0006801] References: PMID:12359750 Sources: GOC:jl Regulation: regulated by regulation of superoxide anion generation [GO:0032928]; negatively regulated by negative regulation of superoxide anion generation [GO:0032929]; positively regulated by positive regulation of superoxide anion generation [GO:0032930] Definition: The enzymatic generation of superoxide, the superoxide anion O2- (superoxide free radical), or any compound containing this species, by a cell in response to environmental stress, thereby mediating the activation of various stress-inducible signaling pathways. Also known as: superoxide release